{
  "term_label": "Unknown molecular function",
  "gene_name": "Putative C-type lectin domain family 20 member A",
  "gene": "UniProtKB:Q6ZU45",
  "gene_symbol": "CLEC20A",
  "term_id": "UNKNOWN:0001"
}